positive regulation of shelterin complex assembly [GO:1904792] (biological process) Also known as: positive regulation of Pot1 complex assembly, positive regulation of Pot1-Tpz1 complex assembly, positive regulation of shelterin complex formation, positive regulation of telosome assembly, up regulation of Pot1 complex assembly, up regulation of Pot1-Tpz1 complex assembly, up regulation of shelterin complex formation, up regulation of telosome assembly, up-regulation of Pot1 complex assembly, up-regulation of Pot1-Tpz1 complex assembly, up-regulation of shelterin complex formation, up-regulation of telosome assembly, upregulation of Pot1 complex assembly, upregulation of Pot1-Tpz1 complex assembly, upregulation of shelterin complex formation, upregulation of telosome assembly, activation of Pot1 complex assembly, activation of Pot1-Tpz1 complex assembly, activation of shelterin complex formation, activation of telosome assembly Relationships: is_a positive regulation of protein-containing complex assembly [GO:0031334]; is a type of regulation of shelterin complex assembly [GO:1904790]; positively regulates shelterin complex assembly [GO:0071573] References: PMID:24270157 Sources: GOC:BHF, GOC:BHF_telomere, GOC:TermGenie, GOC:nc, GO_REF:0000058 Definition: Any process that activates or increases the frequency, rate or extent of shelterin complex assembly.